{
  "gene": "UniProtKB:Q8IY50",
  "term_label": "Unknown molecular function",
  "gene_name": "Solute carrier family 35 member F3",
  "gene_symbol": "SLC35F3",
  "term_id": "UNKNOWN:0001"
}